{
  "term_id": "GO:0000981",
  "term_label": "DNA-binding transcription factor activity, RNA polymerase II-specific",
  "gene_symbol": "FOSL2",
  "gene_name": "Fos-related antigen 2",
  "gene": "UniProtKB:P15408"
}